{
  "gene_name": "Myosin-8",
  "term_id": "GO:0005737",
  "gene": "UniProtKB:P13535",
  "term_label": "cytoplasm",
  "gene_symbol": "MYH8"
}